{
  "gene_symbol": "H1-1",
  "gene": "UniProtKB:Q02539",
  "gene_name": "Histone H1.1",
  "term_label": "double-stranded DNA binding",
  "term_id": "GO:0003690"
}